negative regulation of mRNA catabolic process [GO:1902373] (biological process) Also known as: down regulation of mRNA breakdown, down regulation of mRNA catabolic process, down regulation of mRNA catabolism, down regulation of mRNA degradation, down-regulation of mRNA breakdown, down-regulation of mRNA catabolic process, down-regulation of mRNA catabolism, down-regulation of mRNA degradation, downregulation of mRNA breakdown, downregulation of mRNA catabolic process, downregulation of mRNA catabolism, downregulation of mRNA degradation, negative regulation of mRNA breakdown, negative regulation of mRNA catabolism, negative regulation of mRNA degradation, inhibition of mRNA breakdown, inhibition of mRNA catabolic process, inhibition of mRNA catabolism, inhibition of mRNA degradation, down regulation of mRNA decay, down-regulation of mRNA decay, downregulation of mRNA decay, inhibition of mRNA decay, negative regulation of mRNA decay Definition: Any process that stops, prevents or reduces the frequency, rate or extent of mRNA catabolic process. Subtypes: GO:0048255, negative regulation of deadenylation-dependent decapping of nuclear-transcribed mRNA [GO:0106289], GO:0120271, GO:1900152, GO:1905638, negative regulation of nuclear-transcribed mRNA catabolic process, nonsense-mediated decay [GO:2000623] Relationships: is a type of positive regulation of gene expression [GO:0010628]; is a type of GO:0061013; is a type of negative regulation of RNA catabolic process [GO:1902369]; is a type of negative regulation of mRNA metabolic process [GO:1903312]; negatively regulates mRNA catabolic process [GO:0006402] References: PMID:22626865 Sources: GOC:TermGenie, GOC:bf